{
  "gene": "UniProtKB:Q15628",
  "term_id": "GO:0002947",
  "term_label": "tumor necrosis factor receptor superfamily complex",
  "gene_symbol": "TRADD",
  "gene_name": "Tumor necrosis factor receptor type 1-associated DEATH domain protein"
}